U12-type post-mRNA release spliceosomal complex [GO:0071019] (cellular component) Also known as: minor post-mRNA release spliceosomal complex, AT-AC post-mRNA release spliceosomal complex, mammalian U12-type spliceosomal complex I Relationships: is a type of U12-type spliceosomal complex [GO:0005689]; is a type of post-mRNA release spliceosomal complex [GO:0071014]; has part GO:0005691; has part GO:0005693 References: PMID:16201866 Sources: GOC:ab, GOC:krc, GOC:mah, ISBN:0879695897, ISBN:0879697393 Definition: A spliceosomal complex that is formed following the release of the spliced product from the post-spliceosomal complex and contains the excised intron and the U12, U5 and U6atac snRNPs.